{
  "term_id": "UNKNOWN:0003",
  "gene": "UniProtKB:Q86VW0",
  "term_label": "Unknown cellular component",
  "gene_symbol": "SESTD1",
  "gene_name": "SEC14 domain and spectrin repeat-containing protein 1"
}